{
  "term_id": "GO:0005759",
  "gene_symbol": "HSPE1",
  "gene": "UniProtKB:P61604",
  "gene_name": "10 kDa heat shock protein, mitochondrial",
  "term_label": "mitochondrial matrix"
}